positive regulation of neuronal action potential [GO:1904457] (biological process) Also known as: up regulation of neuronal action potential, up-regulation of neuronal action potential, upregulation of neuronal action potential, activation of neuronal action potential, activation of generation of action potential, positive regulation of generation of action potential, up regulation of generation of action potential, up-regulation of generation of action potential, upregulation of generation of action potential Relationships: is a type of positive regulation of action potential [GO:0045760]; is a type of positive regulation of transmission of nerve impulse [GO:0051971]; is a type of regulation of neuronal action potential [GO:0098908]; positively regulates neuronal action potential [GO:0019228] References: PMID:25126967 Sources: GOC:TermGenie, GO_REF:0000058 Definition: Any process that activates or increases the frequency, rate or extent of neuronal action potential.